tRNA (m7G46) methyltransferase complex [GO:0106143] (cellular component) Relationships: is a type of tRNA methyltransferase complex [GO:0043527] Definition: A protein complex involved in the catalysis of the formation of the modified nucleotide 7-methylguanine (at position 46 in certain tRNAs, such as tRNA(phe) and tRNA(met). In yeast, it is a heterotetramer of two subunits, Trm8 (catalytic) and Trm82 (WD repeat). Also known as: Trm8-Trm82 complex, tRNA (m7G46) methyltransferase, tRNA m7G methylation complex References: PMID:15811913, PMID:1738232, PMID:18164779, PMID:18184583 Sources: GOC:vw